{
  "gene_symbol": "B3GALT6",
  "term_id": "GO:0000139",
  "term_label": "Golgi membrane",
  "gene_name": "Beta-1,3-galactosyltransferase 6",
  "gene": "UniProtKB:Q96L58"
}